{
  "gene_name": "Transcription factor SOX-8",
  "gene": "UniProtKB:P57073",
  "term_id": "GO:0000981",
  "gene_symbol": "SOX8",
  "term_label": "DNA-binding transcription factor activity, RNA polymerase II-specific"
}